{
  "gene": "UniProtKB:Q9BQM9",
  "term_label": "Unknown molecular function",
  "term_id": "UNKNOWN:0001",
  "gene_symbol": "C20orf144",
  "gene_name": "Uncharacterized protein C20orf144"
}